glutaminyl-tRNAGln biosynthesis via transamidation [GO:0070681] (biological process) Sources: GOC:mah, MetaCyc:PWY-5921 Relationships: is a type of GO:0043039 Definition: A tRNA aminoacylation process in which glutaminyl-tRNAGln is formed by a tRNA-dependent two-step pathway. In the first step a non-discriminating glutamyl-tRNAGlx synthetase generates the misacylated L-glutamyl-tRNAGln species, and in the second step it is amidated to the correctly charged L-glutaminyl-tRNAGln by a glutamyl-tRNAGln amidotransferase.